{
  "term_label": "nucleus",
  "gene_symbol": "PRR11",
  "gene_name": "Proline-rich protein 11",
  "term_id": "GO:0005634",
  "gene": "UniProtKB:Q96HE9"
}